carbamoyl-phosphate synthase complex [GO:0005951] (cellular component) References: PMID:8626695 Also known as: carbamoyl phosphate synthase complex, arginine-specific carbamoyl phosphate synthetase complex, carbamoyl-phosphate synthase arginine-specific complex Definition: A protein complex that catalyzes the formation of carbamoyl phosphate; comprises a small subunit that binds and cleaves glutamine, and a large subunit that accepts the ammonia group cleaved from glutamine, binds all of the remaining substrates and effectors, and carries out all of the other catalytic events. Note: Note that in higher eukaryotes, carbamoyl-phosphate synthase is usually a single polypeptide, not a complex, and should therefore not be annotated to this component term. Relationships: is a type of catalytic complex [GO:1902494]; is part of cytoplasm [GO:0005737]